{
  "term_label": "positive regulation of systemic arterial blood pressure",
  "term_id": "GO:0003084",
  "gene_name": "Vasopressin-neurophysin 2-copeptin",
  "gene_symbol": "AVP",
  "gene": "UniProtKB:P01185"
}